deacylase activity [GO:0160215] (molecular function) Definition: Catalysis of the reaction: R-CO-X + H2O = R-COOH + HX, hydrolysis of an acyl group or groups from a substrate molecule. Subtypes: aminoacyl-tRNA deacylase activity [GO:0002161], acyl-CoA hydrolase activity [GO:0016289], deacetylase activity [GO:0019213], NAD-dependent protein lysine deacylase activity [GO:0141218], protein lysine delactylase activity [GO:0160216] References: PMID:2760018, PMID:29637793, PMID:38355760 Relationships: is a type of catalytic activity [GO:0003824]